{
  "gene_symbol": "CLTC",
  "gene_name": "Clathrin heavy chain 1",
  "term_label": "receptor-mediated endocytosis",
  "gene": "UniProtKB:Q00610",
  "term_id": "GO:0006898"
}